{
  "gene_name": "Olfactory receptor 6N1",
  "gene": "UniProtKB:Q8NGY5",
  "term_id": "GO:0005886",
  "term_label": "plasma membrane",
  "gene_symbol": "OR6N1"
}